trimethyluric acid monooxygenase activity [GO:0102613] (molecular function) Relationships: is a type of oxidoreductase activity, acting on paired donors, with incorporation or reduction of molecular oxygen, NAD(P)H as one donor, and incorporation of one atom of oxygen [GO:0016709] Sources: GOC:pz, RHEA:48992 Definition: Catalysis of the reaction: 1,3,7-trimethyluric acid + O2 + NADH + 3 H+ = 1,3,7-trimethyl-5-hydroxyisourate + NAD + H2O.